{
  "gene": "UniProtKB:Q5VT52",
  "term_label": "Unknown cellular component",
  "term_id": "UNKNOWN:0003",
  "gene_symbol": "RPRD2",
  "gene_name": "Regulation of nuclear pre-mRNA domain-containing protein 2"
}